mCRD-mediated mRNA stability complex [GO:0106002] (CC) Definition: A protein complex that binds to, and promotes stabilization of, mRNA molecules containing the major coding region instability determinant (mCRD) by bridging the mCRD domain and the poly(A) tail of the mRNA. In human, it consists of CSDE1, HNRPD, PABPC1, PAIP1 and SYNCRIP. Also known as: mCRD-poly(A)-bridging complex, major coding region determinant of instability-mediated mRNA stability complex, major coding region instability determinant-mediated mRNA stability complex, major coding region instability determinant-poly(A)-bridging complex, major coding-region determinant of instability - poly(A) tail-bridging complex Relationships: is a type of GO:0032991; is part of cytosol [GO:0005829] Note: This complex is related to GO:0070937 CRD-mediated mRNA stability complex but binds the major protein-coding-region determinant of instability (mCRD) domain rather than the CRD. Experimentally it has been shown to act on c-FOS mRNA while GO:0070937 acts on c-MYC mRNA. References: PMID:11051545 Sources: GOC:bhm